{
  "gene_name": "Putative 3-phosphoinositide-dependent protein kinase 2",
  "term_label": "insulin receptor signaling pathway",
  "gene_symbol": "PDPK2P",
  "gene": "UniProtKB:Q6A1A2",
  "term_id": "GO:0008286"
}